{
  "term_id": "GO:0045087",
  "gene": "UniProtKB:Q6P9F5",
  "gene_name": "E3 ubiquitin ligase TRIM40",
  "gene_symbol": "TRIM40",
  "term_label": "innate immune response"
}